extracellular ammonia-gated monoatomic ion channel activity [GO:0036081] (molecular function) References: PMID:19135896 Sources: GOC:sart Relationships: is a type of extracellular ligand-gated monoatomic ion channel activity [GO:0005230] Definition: Enables the transmembrane transfer of an ion by a channel that opens when extracellular ammonia (NH3) has been bound by the channel complex or one of its constituent parts. Also known as: extracellular ammonia-gated ion channel activity, ionotropic ammonia receptor activity